{
  "gene_symbol": "ZNF805",
  "gene_name": "Zinc finger protein 805",
  "gene": "UniProtKB:Q5CZA5",
  "term_label": "RNA polymerase II cis-regulatory region sequence-specific DNA binding",
  "term_id": "GO:0000978"
}